{
  "gene_name": "Immunoglobulin heavy variable 4-39",
  "gene_symbol": "IGHV4-39",
  "gene": "UniProtKB:P01824",
  "term_label": "Unknown cellular component",
  "term_id": "UNKNOWN:0003"
}